{
  "gene_symbol": "GPR119",
  "gene_name": "Glucose-dependent insulinotropic receptor",
  "term_id": "GO:0004930",
  "term_label": "G protein-coupled receptor activity",
  "gene": "UniProtKB:Q8TDV5"
}